{
  "gene": "UniProtKB:Q96SQ7",
  "term_id": "GO:0005634",
  "gene_symbol": "ATOH8",
  "gene_name": "Transcription factor ATOH8",
  "term_label": "nucleus"
}